{
  "term_id": "GO:0038048",
  "gene": "UniProtKB:P41145",
  "gene_name": "Kappa-type opioid receptor",
  "term_label": "dynorphin receptor activity",
  "gene_symbol": "OPRK1"
}